lactate racemase activity [GO:0050043] (molecular function) Definition: Catalysis of the reaction: (S)-lactate = (R)-lactate. Relationships: is a type of racemase and epimerase activity, acting on hydroxy acids and derivatives [GO:0016856] Also known as: hydroxyacid racemase activity, lactic acid racemase activity, lacticoracemase activity Sources: EC:5.1.2.1, RHEA:10960